{
  "term_id": "GO:0005516",
  "gene_symbol": "MAPKAPK3",
  "gene": "UniProtKB:Q16644",
  "gene_name": "MAP kinase-activated protein kinase 3",
  "term_label": "calmodulin binding"
}